DnaB-DnaG complex [GO:1990156] (cellular component) References: PMID:14557266 Sources: GOC:bhm Relationships: is a type of DNA helicase complex [GO:0033202]; is part of core primosome complex [GO:1990098]; has part DnaB helicase complex [GO:1990161] Also known as: DnaB-DnaG primosome complex Definition: A protein complex containing homohexameric DnaB helicase, and DnaG (a primase). Facilitates the unwinding of double-stranded DNA and the synthesis of RNA primer sequences during DNA replication and repair in Prokaryotes.